{
  "gene": "UniProtKB:A0A1B0GV96",
  "gene_name": "CHD9 neighbor protein",
  "term_id": "UNKNOWN:0001",
  "gene_symbol": "CHD9NB",
  "term_label": "Unknown molecular function"
}